transposable element silencing by piRNA-mediated heterochromatin formation [GO:0141006] (biological process) Relationships: is a type of piRNA-mediated heterochromatin formation [GO:0140966]; is a type of transposable element silencing by heterochromatin formation [GO:0141005] Definition: A transposable element silencing mechanism in which a Piwi-associated RNA (piRNA) triggers heterochromatin assembly. Heterochromatin is a chromatin conformation that is refractory to transcription. Also known as: piRNA-mediated retrotransposon silencing by heterochromatin formation References: PMID:32381626, PMID:32674113